4-hydroxycyclohexanecarboxylate dehydrogenase activity [GO:0047030] (molecular function) Also known as: trans-4-hydroxycyclohexanecarboxylate dehydrogenase activity, trans-4-hydroxycyclohexanecarboxylate:NAD+ 4-oxidoreductase activity Sources: EC:1.1.1.226, RHEA:17429 Relationships: is a type of oxidoreductase activity, acting on the CH-OH group of donors, NAD or NADP as acceptor [GO:0016616] Definition: Catalysis of the reaction: trans-4-hydroxycyclohexanecarboxylate + NAD+ = 4-oxocyclohexanecarboxylate + H+ + NADH.